{
  "term_label": "protein phosphatase type 1 complex",
  "gene_name": "Protein phosphatase 1 regulatory subunit 3A",
  "term_id": "GO:0000164",
  "gene": "UniProtKB:Q16821",
  "gene_symbol": "PPP1R3A"
}